{
  "gene_name": "Protein PROCA1",
  "term_label": "Unknown biological process",
  "gene": "UniProtKB:Q8NCQ7",
  "gene_symbol": "PROCA1",
  "term_id": "UNKNOWN:0002"
}